inositol-1,5-bisdiphosphate-2,3,4,6-tetrakisphosphate 5-diphosphatase activity [GO:0052847] (molecular function) References: PMID:10827188, PMID:11502751 Sources: MetaCyc:RXN-10975 Definition: Catalysis of the reaction: 1,5-bisdiphospho-1D-myo-inositol 2,3,4,6-tetrakisphosphate + H2O = 1-diphospho-1D-myo-inositol 2,3,4,5,6-pentakisphosphate + phosphate + H+. Relationships: is a type of inositol bisdiphosphate tetrakisphosphate diphosphatase activity [GO:0052841]